3'-5'-exoribonuclease activity involved in mature miRNA 3'-end processing [GO:0044748] (molecular function) Relationships: is a type of 3'-5'-RNA exonuclease activity [GO:0000175]; is part of pre-miRNA 3'-end processing [GO:0044747] Also known as: exonucleolytic trimming to generate 3' end of miRNA Definition: Catalysis of the sequential cleavage of mononucleotides from a free 3' terminus of an RNA molecule that contributes to forming distinct miRNA isoforms from a mature miRNA. Sources: GOC:sart